{
  "gene_name": "TGF-beta-activated kinase 1 and MAP3K7-binding protein 3",
  "term_id": "UNKNOWN:0001",
  "gene": "UniProtKB:Q8N5C8",
  "gene_symbol": "TAB3",
  "term_label": "Unknown molecular function"
}